{
  "term_id": "GO:0001228",
  "term_label": "DNA-binding transcription activator activity, RNA polymerase II-specific",
  "gene_name": "Histone-lysine N-methyltransferase PRDM16",
  "gene_symbol": "PRDM16",
  "gene": "UniProtKB:Q9HAZ2"
}